{
  "gene": "UniProtKB:Q8WWI1",
  "term_label": "Unknown molecular function",
  "gene_symbol": "LMO7",
  "gene_name": "LIM domain only protein 7",
  "term_id": "UNKNOWN:0001"
}